alpha-2C adrenergic receptor binding [GO:0031696] (molecular function) Definition: Binding to an alpha-2C adrenergic receptor. Sources: GOC:mah, GOC:nln Also known as: alpha-2C adrenergic receptor ligand Relationships: is a type of adrenergic receptor binding [GO:0031690]